2-oxobutyrate synthase activity [GO:0018491] (MF) Definition: Catalysis of the reaction: 2-oxobutanoate + CoA + oxidized ferredoxin = propanoyl-CoA + CO2 + reduced ferredoxin. Sources: GOC:curators Also known as: 2-ketobutyrate synthase activity, 2-oxobutanoate:ferredoxin 2-oxidoreductase (CoA-propionylating), 2-oxobutyrate-ferredoxin oxidoreductase activity, alpha-ketobutyrate synthase activity, alpha-ketobutyrate-ferredoxin oxidoreductase activity Relationships: is a type of GO:0016620